{
  "term_id": "UNKNOWN:0002",
  "gene_name": "Golgi resident protein GCP60",
  "term_label": "Unknown biological process",
  "gene": "UniProtKB:Q9H3P7",
  "gene_symbol": "ACBD3"
}